{
  "gene_symbol": "PRSS3P2",
  "term_label": "proteolysis",
  "gene": "UniProtKB:Q8NHM4",
  "term_id": "GO:0006508",
  "gene_name": "Putative trypsin-6"
}